{
  "gene_name": "Ligand of Numb protein X 2",
  "term_label": "ubiquitin-protein transferase activity",
  "gene_symbol": "LNX2",
  "gene": "UniProtKB:Q8N448",
  "term_id": "GO:0004842"
}